{
  "term_id": "GO:0005886",
  "gene": "UniProtKB:P21731",
  "term_label": "plasma membrane",
  "gene_name": "Thromboxane A2 receptor",
  "gene_symbol": "TBXA2R"
}